{
  "gene": "UniProtKB:A0A075B6K4",
  "gene_name": "Immunoglobulin lambda variable 3-10",
  "term_label": "immune response",
  "term_id": "GO:0006955",
  "gene_symbol": "IGLV3-10"
}